{
  "term_label": "RNA polymerase II cis-regulatory region sequence-specific DNA binding",
  "gene": "UniProtKB:O43248",
  "term_id": "GO:0000978",
  "gene_symbol": "HOXC11",
  "gene_name": "Homeobox protein Hox-C11"
}